{
  "gene": "UniProtKB:P15374",
  "gene_name": "Ubiquitin carboxyl-terminal hydrolase isozyme L3",
  "term_id": "GO:0005737",
  "gene_symbol": "UCHL3",
  "term_label": "cytoplasm"
}